{
  "term_id": "UNKNOWN:0001",
  "term_label": "Unknown molecular function",
  "gene_symbol": "CCDC17",
  "gene": "UniProtKB:Q96LX7",
  "gene_name": "Coiled-coil domain-containing protein 17"
}